mitochondrial tyrosyl-tRNA aminoacylation [GO:0070184] (biological process) Definition: The process of coupling tyrosine to tyrosyl-tRNA in a mitochondrion, catalyzed by tyrosyl-tRNA synthetase. In tRNA aminoacylation, the amino acid is first activated by linkage to AMP and then transferred to either the 2'- or the 3'-hydroxyl group of the 3'-adenosine residue of the tRNA. Sources: GOC:mah, GOC:mcc Relationships: is a type of tyrosyl-tRNA aminoacylation [GO:0006437]; is a type of tRNA aminoacylation for mitochondrial protein translation [GO:0070127]